{
  "gene": "UniProtKB:Q96G21",
  "gene_symbol": "IMP4",
  "gene_name": "U3 small nucleolar ribonucleoprotein protein IMP4",
  "term_id": "GO:0032040",
  "term_label": "small-subunit processome"
}